(2E)-butenoyl-CoA hydratase activity [GO:0120092] (molecular function) Definition: Catalysis of the reaction: 3-hydroxybutanoyl-CoA = (2E)-butenoyl-CoA + H2O. (2E)-butenoyl-CoA is also known as crotonoyl-CoA. References: PMID:28803779 Sources: RHEA:45584 Also known as: crotonyl-CoA hydratase activity Relationships: is a type of 3-hydroxyacyl-CoA dehydratase activity [GO:0018812]